{
  "gene_symbol": "P0DMU3",
  "term_id": "UNKNOWN:0003",
  "gene_name": "FAM231A_C-like protein LOC102723383",
  "gene": "UniProtKB:P0DMU3",
  "term_label": "Unknown cellular component"
}